{
  "gene_name": "Protein tyrosine phosphatase type IVA 3",
  "term_label": "protein tyrosine phosphatase activity",
  "term_id": "GO:0004725",
  "gene": "UniProtKB:O75365",
  "gene_symbol": "PTP4A3"
}